{
  "gene": "UniProtKB:Q15700",
  "term_label": "protein kinase binding",
  "term_id": "GO:0019901",
  "gene_symbol": "DLG2",
  "gene_name": "Disks large homolog 2"
}